extracellular phenylacetaldehyde-gated monoatomic ion channel activity [GO:0036082] (molecular function) Also known as: extracellular phenylacetaldehyde-gated ion channel activity, ionotropic phenylacetaldehyde receptor activity Definition: Enables the transmembrane transfer of an ion by a channel that opens when extracellular phenylacetaldehyde has been bound by the channel complex or one of its constituent parts. References: PMID:19135896 Sources: GOC:sart Relationships: is a type of extracellular ligand-gated monoatomic ion channel activity [GO:0005230]